negative regulation of division septum assembly [GO:0010974] (biological process) Definition: Any process that decreases the frequency, rate or extent of division septum formation. division septum formation is he assembly and arrangement of a septum that spans the plasma membrane interface between progeny cells following cytokinesis. Relationships: is a type of regulation of division septum assembly [GO:0032955]; is a type of negative regulation of cell septum assembly [GO:1901892]; negatively regulates division septum assembly [GO:0000917] Also known as: negative regulation of division septum formation, inhibition of division septum assembly involved in cell cycle cytokinesis References: PMID:19959363, PMID:21246752, PMID:22786806 Sources: GOC:mtg_cell_cycle Subtypes: GO:0031030, negative regulation of mitotic division septum assembly [GO:0140280]